{
  "gene_name": "Zinc finger protein 888",
  "gene_symbol": "ZNF888",
  "term_id": "GO:0005634",
  "gene": "UniProtKB:P0CJ79",
  "term_label": "nucleus"
}